{
  "gene": "UniProtKB:Q9NUE0",
  "term_label": "endoplasmic reticulum",
  "gene_name": "Palmitoyltransferase ZDHHC18",
  "gene_symbol": "ZDHHC18",
  "term_id": "GO:0005783"
}